N-acetyllactosaminide alpha-2,3-sialyltransferase activity [GO:0008118] (molecular function) Relationships: is a type of sialyltransferase activity [GO:0008373] Definition: Catalysis of the reaction: a beta-D-galactosyl-(1->4)-N-acetyl-beta-D-glucosaminyl derivative + CMP-N-acetyl-beta-neuraminate = an N-acetyl-alpha-neuraminyl-(2->3)-beta-D-galactosyl-(1->4)-N-acetyl-beta-D-glucosaminyl derivative + CMP + H+. Note: The substrate for this reaction is a beta-D-galactosyl-(1->4)-N-acetyl- D-glucosaminyl (known as type 2 histo-blood group precursor disaccharide) in non-reducing termini of glycan moieties in glycoproteins and glycolipids. References: PMID:10206952 Sources: RHEA:52316 Also known as: N-acetyllactosaminide alpha-2,3-sialyltransferase, neolactotetraosylceramide alpha-2,3-sialyltransferase activity, alpha2->3 sialyltransferase activity, cytidine monophosphoacetylneuraminate-beta-galactosyl(1->4)acetylglucosaminide alpha2->3-sialyltransferase activity